{
  "term_id": "UNKNOWN:0001",
  "gene_name": "Ran-binding protein 3-like",
  "term_label": "Unknown molecular function",
  "gene_symbol": "RANBP3L",
  "gene": "UniProtKB:Q86VV4"
}